{
  "gene_symbol": "TBC1D4",
  "term_id": "GO:0005096",
  "gene_name": "TBC1 domain family member 4",
  "term_label": "GTPase activator activity",
  "gene": "UniProtKB:O60343"
}